negative regulation of hematopoietic stem cell differentiation [GO:1902037] (biological process) References: PMID:23403623 Sources: GOC:TermGenie Relationships: is a type of negative regulation of hematopoietic progenitor cell differentiation [GO:1901533]; is a type of regulation of hematopoietic stem cell differentiation [GO:1902036]; is a type of GO:2000737; negatively regulates hematopoietic stem cell differentiation [GO:0060218] Definition: Any process that stops, prevents or reduces the frequency, rate or extent of hematopoietic stem cell differentiation. Also known as: down regulation of haematopoietic stem cell differentiation, down regulation of haemopoietic stem cell differentiation, down regulation of hematopoietic stem cell differentiation, down regulation of hemopoietic stem cell differentiation, down-regulation of haematopoietic stem cell differentiation, down-regulation of haemopoietic stem cell differentiation, down-regulation of hematopoietic stem cell differentiation, down-regulation of hemopoietic stem cell differentiation, downregulation of haematopoietic stem cell differentiation, downregulation of haemopoietic stem cell differentiation, downregulation of hematopoietic stem cell differentiation, downregulation of hemopoietic stem cell differentiation, negative regulation of haematopoietic stem cell differentiation, negative regulation of haemopoietic stem cell differentiation, negative regulation of hemopoietic stem cell differentiation, inhibition of haematopoietic stem cell differentiation, inhibition of haemopoietic stem cell differentiation, inhibition of hematopoietic stem cell differentiation, inhibition of hemopoietic stem cell differentiation